{
  "gene_symbol": "TBC1D25",
  "term_label": "regulation of autophagosome maturation",
  "term_id": "GO:1901096",
  "gene_name": "TBC1 domain family member 25",
  "gene": "UniProtKB:Q3MII6"
}